{
  "gene_name": "17-beta-hydroxysteroid dehydrogenase type 2",
  "gene_symbol": "HSD17B2",
  "term_label": "Unknown cellular component",
  "gene": "UniProtKB:P37059",
  "term_id": "UNKNOWN:0003"
}